{
  "term_label": "cargo receptor activity",
  "term_id": "GO:0038024",
  "gene_symbol": "AMN",
  "gene_name": "Protein amnionless",
  "gene": "UniProtKB:Q9BXJ7"
}